vesicle docking [GO:0048278] (biological process) Relationships: is a type of organelle localization by membrane tethering [GO:0140056]; is part of vesicle-mediated transport [GO:0016192] Sources: GOC:ai, GOC:jid Also known as: vesicle to membrane docking Subtypes: vesicle docking involved in exocytosis [GO:0006904], GO:0048211, phagosome-lysosome docking [GO:0090384] Regulation: regulated by regulation of vesicle docking [GO:0106020]; negatively regulated by negative regulation of vesicle docking [GO:0106021]; RO_0002213 by positive regulation of vesicle docking [GO:0106022] Definition: The initial attachment of a transport vesicle membrane to the target membrane, mediated by proteins protruding from the membrane of the vesicle and the target membrane. Docking requires only that the two membranes come close enough for these proteins to interact and adhere.